{
  "gene_symbol": "IL1RAPL1",
  "term_label": "cell surface receptor signaling pathway",
  "gene_name": "Interleukin-1 receptor accessory protein-like 1",
  "term_id": "GO:0007166",
  "gene": "UniProtKB:Q9NZN1"
}